circumferential growth involved in left ventricle morphogenesis [GO:0003243] (biological process) Definition: The morphogenetic growth in which the left ventricle grows expanding its external boundary. References: PMID:14709543 Sources: GOC:mtg_heart Relationships: is_a GO:0003241; is part of GO:0003214